glutamate formimidoyltransferase activity [GO:0030409] (molecular function) Sources: RHEA:15097 Relationships: is a type of hydroxymethyl-, formyl- and related transferase activity [GO:0016742] Definition: Catalysis of the reaction: 5-formimidoyltetrahydrofolate + L-glutamate = tetrahydrofolate + N-formimidoyl-L-glutamate. Also known as: formimidoyltransferase activity, formiminotransferase activity, glutamate formiminotransferase activity, 5-formimidoyltetrahydrofolate:L-glutamate N-formimidoyltransferase activity, formiminoglutamic acid transferase activity, formiminoglutamic formiminotransferase activity, glutamate formyltransferase activity